{
  "term_label": "vesicle-mediated transport",
  "gene": "UniProtKB:Q6XYQ8",
  "gene_symbol": "SYT10",
  "gene_name": "Synaptotagmin-10",
  "term_id": "GO:0016192"
}